{
  "gene": "UniProtKB:Q9H237",
  "gene_name": "Protein-serine O-palmitoleoyltransferase porcupine",
  "gene_symbol": "PORCN",
  "term_id": "GO:0017147",
  "term_label": "Wnt-protein binding"
}